{
  "term_id": "UNKNOWN:0002",
  "term_label": "Unknown biological process",
  "gene_name": "Putative uncharacterized protein ZNF516-DT",
  "gene": "UniProtKB:Q6ZTR6",
  "gene_symbol": "ZNF516-DT"
}